{
  "term_id": "GO:0042867",
  "gene": "UniProtKB:P07195",
  "term_label": "pyruvate catabolic process",
  "gene_name": "L-lactate dehydrogenase B chain",
  "gene_symbol": "LDHB"
}